{
  "gene_name": "cAMP-regulated phosphoprotein 19",
  "term_label": "cytoplasm",
  "term_id": "GO:0005737",
  "gene_symbol": "ARPP19",
  "gene": "UniProtKB:P56211"
}